{
  "term_id": "UNKNOWN:0003",
  "gene_name": "COMM domain-containing protein 3",
  "gene": "UniProtKB:Q9UBI1",
  "term_label": "Unknown cellular component",
  "gene_symbol": "COMMD3"
}